lytic endotransglycosylase activity [GO:0008932] (molecular function) Definition: Catalysis of the endolytic cleavage of the (1->4)-beta-glycosidic linkage between N-acetylmuramic acid (MurNAc) and N-acetylglucosamine (GlcNAc) residues in peptidoglycan with concomitant formation of a 1,6-anhydrobond in the MurNAc residue. Also known as: murein lytic endotransglycosylase E activity References: PMID:10964424, PMID:9642199 Sources: EC:4.2.2.n2 Relationships: is a type of GO:0008933